{
  "gene": "UniProtKB:Q15019",
  "term_label": "septin complex",
  "gene_symbol": "SEPTIN2",
  "gene_name": "Septin-2",
  "term_id": "GO:0031105"
}